{
  "gene_symbol": "KRT14",
  "gene_name": "Keratin, type I cytoskeletal 14",
  "gene": "UniProtKB:P02533",
  "term_label": "cytoskeleton",
  "term_id": "GO:0005856"
}